FAL1-SGD1 complex [GO:0097078] (CC) References: PMID:21576267 Sources: GOC:rb Definition: A protein complex involved in the 18S rRNA biogenesis. In S. cerevisiae this complex consists of Fal1p and Sgd1p and in humans this complex consists of NOM1 and eIF4AIII subunits. Relationships: is a type of GO:0032991